{
  "term_id": "GO:0005634",
  "gene_symbol": "WBP2",
  "gene": "UniProtKB:Q969T9",
  "gene_name": "WW domain-binding protein 2",
  "term_label": "nucleus"
}